{
  "term_label": "mRNA 5'-splice site recognition",
  "gene": "UniProtKB:P09234",
  "term_id": "GO:0000395",
  "gene_symbol": "SNRPC",
  "gene_name": "U1 small nuclear ribonucleoprotein C"
}